{
  "term_label": "double-stranded RNA binding",
  "gene_symbol": "ZFR2",
  "gene_name": "Zinc finger RNA-binding protein 2",
  "gene": "UniProtKB:Q9UPR6",
  "term_id": "GO:0003725"
}